kaempferol 3-O-galactosyltransferase activity [GO:0033834] (molecular function) Sources: RHEA:15709 Relationships: is a type of hexosyltransferase activity [GO:0016758] Definition: Catalysis of the reaction: UDP-galactose + kaempferol = UDP + kaempferol 3-O-beta-D-galactoside. Also known as: F3GalTase activity, UDP-galactose:kaempferol 3-O-beta-D-galactosyltransferase activity